extrinsic component of plastid thylakoid membrane [GO:0035449] (cellular component) Relationships: is a type of GO:0035448; is a type of extrinsic component of plastid membrane [GO:0035452]; is part of plastid thylakoid membrane [GO:0055035] Subtypes: extrinsic component of lumenal side of plastid thylakoid membrane [GO:0035450], extrinsic component of stromal side of plastid thylakoid membrane [GO:0035451] Sources: GOC:bf, GOC:dos Definition: The component of a plastid thylakoid membrane consisting of gene products and protein complexes that are loosely bound to one of its surfaces, but not integrated into the hydrophobic region. Also known as: peripheral to plastid thylakoid membrane, extrinsic to plastid thylakoid membrane